{
  "gene_name": "GPI transamidase component PIG-S",
  "term_label": "attachment of GPI anchor to protein",
  "gene_symbol": "PIGS",
  "gene": "UniProtKB:Q96S52",
  "term_id": "GO:0016255"
}